{
  "term_id": "GO:0005634",
  "gene_symbol": "FSBP",
  "term_label": "nucleus",
  "gene_name": "Fibrinogen silencer-binding protein",
  "gene": "UniProtKB:O95073"
}